{
  "term_label": "Unknown molecular function",
  "term_id": "UNKNOWN:0001",
  "gene_symbol": "WDR72",
  "gene": "UniProtKB:Q3MJ13",
  "gene_name": "WD repeat-containing protein 72"
}